RISC complex binding [GO:1905172] (molecular function) Relationships: is_a GO:0043021 Definition: Binding to a RISC complex. References: PMID:24882364 Sources: GOC:PARL, GOC:TermGenie, GOC:bf Also known as: RNA-induced silencing complex binding